{
  "term_id": "GO:0001228",
  "gene_symbol": "ZFX",
  "term_label": "DNA-binding transcription activator activity, RNA polymerase II-specific",
  "gene": "UniProtKB:P17010",
  "gene_name": "Zinc finger X-chromosomal protein"
}